{
  "term_id": "GO:0005471",
  "gene": "UniProtKB:P12235",
  "gene_name": "ADP_ATP translocase 1",
  "gene_symbol": "SLC25A4",
  "term_label": "ATP:ADP antiporter activity"
}